{
  "term_label": "endocytosis",
  "gene_symbol": "ATP9A",
  "gene_name": "Probable phospholipid-transporting ATPase IIA",
  "gene": "UniProtKB:O75110",
  "term_id": "GO:0006897"
}